{
  "gene_symbol": "TRUB1",
  "term_id": "GO:1990481",
  "gene_name": "Pseudouridylate synthase TRUB1",
  "term_label": "mRNA pseudouridine synthesis",
  "gene": "UniProtKB:Q8WWH5"
}